{
  "gene": "UniProtKB:Q6NVV1",
  "gene_symbol": "RPL13AP3",
  "term_label": "Unknown cellular component",
  "term_id": "UNKNOWN:0003",
  "gene_name": "Putative ribosomal protein uL13-like"
}